{
  "gene_name": "Bardet-Biedl syndrome 5 protein",
  "term_id": "GO:0032266",
  "gene": "UniProtKB:Q8N3I7",
  "term_label": "phosphatidylinositol-3-phosphate binding",
  "gene_symbol": "BBS5"
}